{
  "gene": "UniProtKB:Q14680",
  "term_id": "UNKNOWN:0002",
  "gene_symbol": "MELK",
  "term_label": "Unknown biological process",
  "gene_name": "Maternal embryonic leucine zipper kinase"
}